{
  "gene_name": "Histone H2B type 1-J",
  "gene": "UniProtKB:P06899",
  "term_id": "GO:0030527",
  "gene_symbol": "H2BC11",
  "term_label": "structural constituent of chromatin"
}